{
  "gene": "UniProtKB:Q9GZV9",
  "gene_name": "Fibroblast growth factor 23",
  "term_label": "extracellular space",
  "gene_symbol": "FGF23",
  "term_id": "GO:0005615"
}